cyanate catabolic process [GO:0009440] (biological process) Definition: The chemical reactions and pathways resulting in the breakdown of cyanate, NCO-, the anion of cyanic acid. Sources: ISBN:0198506732 Also known as: cyanate breakdown, cyanate catabolism, cyanate degradation Relationships: is a type of catabolic process [GO:0009056]